{
  "term_label": "immune response",
  "gene_symbol": "CXCR3",
  "gene_name": "C-X-C chemokine receptor type 3",
  "term_id": "GO:0006955",
  "gene": "UniProtKB:P49682"
}